{
  "gene_symbol": "NRG2",
  "term_label": "signaling receptor binding",
  "gene": "UniProtKB:O14511",
  "gene_name": "Pro-neuregulin-2, membrane-bound isoform",
  "term_id": "GO:0005102"
}